{
  "gene_symbol": "MTA2",
  "term_id": "GO:0016581",
  "gene": "UniProtKB:O94776",
  "gene_name": "Metastasis-associated protein MTA2",
  "term_label": "NuRD complex"
}